{
  "gene_symbol": "SLC25A15",
  "term_id": "GO:0000064",
  "gene": "UniProtKB:Q9Y619",
  "gene_name": "Mitochondrial ornithine transporter 1",
  "term_label": "L-ornithine transmembrane transporter activity"
}